{
  "gene": "UniProtKB:Q92502",
  "term_label": "Unknown cellular component",
  "gene_symbol": "STARD8",
  "gene_name": "StAR-related lipid transfer protein 8",
  "term_id": "UNKNOWN:0003"
}